{
  "gene": "UniProtKB:Q14590",
  "gene_symbol": "ZNF235",
  "term_label": "Unknown molecular function",
  "term_id": "UNKNOWN:0001",
  "gene_name": "Zinc finger protein 235"
}